inhibition of neurotransmitter uptake [GO:0051609] (biological process) Definition: Any process that prevents the activation of the directed movement of a neurotransmitter into a cell. Sources: GOC:ai Also known as: inhibition of neurotransmitter import Relationships: is a type of negative regulation of neurotransmitter uptake [GO:0051581] Subtypes: inhibition of dopamine uptake involved in synaptic transmission [GO:0051587], inhibition of serotonin uptake [GO:0051614], inhibition of histamine uptake [GO:0051619], inhibition of norepinephrine uptake [GO:0051624], inhibition of epinephrine uptake [GO:0051629], inhibition of acetylcholine uptake [GO:0051634]